{
  "gene_symbol": "TRBV12-3",
  "term_label": "plasma membrane",
  "term_id": "GO:0005886",
  "gene_name": "T cell receptor beta variable 12-3",
  "gene": "UniProtKB:P01733"
}